{
  "term_id": "GO:0042127",
  "gene_symbol": "SMIM22",
  "term_label": "regulation of cell population proliferation",
  "gene": "UniProtKB:K7EJ46",
  "gene_name": "Small integral membrane protein 22"
}